positive regulation of NLRP3 inflammasome complex assembly [GO:1900227] (BP) Definition: Any process that activates or increases the frequency, rate or extent of NLRP3 inflammasome complex assembly. Sources: GOC:TermGenie Also known as: activation of NALP3 inflammasome complex assembly, positive regulation of NALP3 inflammasome complex assembly, up regulation of NALP3 inflammasome complex assembly, up regulation of NLRP3 inflammasome complex assembly, up-regulation of NALP3 inflammasome complex assembly, up-regulation of NLRP3 inflammasome complex assembly, upregulation of NALP3 inflammasome complex assembly, upregulation of NLRP3 inflammasome complex assembly, activation of NLRP3 inflammasome complex assembly, activation of NLRP3 inflammasome activation, positive regulation of NLRP3 inflammasome activation, up regulation of NLRP3 inflammasome activation, up-regulation of NLRP3 inflammasome activation, upregulation of NLRP3 inflammasome activation Relationships: is a type of GO:0031334; is_a regulation of NLRP3 inflammasome complex assembly [GO:1900225]; is part of positive regulation of inflammasome-mediated signaling pathway [GO:0141087]; positively regulates GO:0044546